{
  "term_label": "Unknown molecular function",
  "gene": "UniProtKB:A6NJY1",
  "gene_name": "Putative SLC9B1-like protein SLC9B1P1",
  "term_id": "UNKNOWN:0001",
  "gene_symbol": "SLC9B1P1"
}